{
  "gene_name": "Phosphorylase b kinase gamma catalytic chain, liver_testis isoform",
  "gene": "UniProtKB:P15735",
  "term_id": "GO:0004689",
  "term_label": "phosphorylase kinase activity",
  "gene_symbol": "PHKG2"
}